biofilm matrix organization [GO:0098784] (biological process) Sources: GOC:mah Subtypes: biofilm matrix assembly [GO:0098785], biofilm matrix disassembly [GO:0098786] Definition: A process that results in the assembly, arrangement of constituent parts, or disassembly of a biofilm matrix. Relationships: is a type of extracellular matrix organization [GO:0030198] Also known as: biofilm matrix organization and biogenesis